intrinsic apoptotic signaling pathway in response to DNA damage by p53 class mediator [GO:0042771] (biological process) Relationships: is_a GO:0008630; is a type of intrinsic apoptotic signaling pathway by p53 class mediator [GO:0072332] Definition: The series of molecular signals in which an intracellular signal is conveyed to trigger the apoptotic death of a cell. The pathway is induced by the cell cycle regulator phosphoprotein p53, or an equivalent protein, in response to the detection of DNA damage, and ends when the execution phase of apoptosis is triggered. Also known as: DNA damage response, signal transduction by p53 class mediator resulting in induction of apoptosis Sources: GOC:go_curators, GOC:mtg_apoptosis Regulation: regulated by regulation of intrinsic apoptotic signaling pathway in response to DNA damage by p53 class mediator [GO:1902165]; negatively regulated by negative regulation of intrinsic apoptotic signaling pathway in response to DNA damage by p53 class mediator [GO:1902166]; positively regulated by positive regulation of intrinsic apoptotic signaling pathway in response to DNA damage by p53 class mediator [GO:1902167]